{
  "term_label": "Unknown cellular component",
  "gene_symbol": "ASDURF",
  "gene_name": "ASNSD1 upstream open reading frame protein",
  "gene": "UniProtKB:L0R819",
  "term_id": "UNKNOWN:0003"
}